isoflavonoid phytoalexin biosynthetic process [GO:0009701] (biological process) Definition: The chemical reactions and pathways resulting in the formation of isoflavonoid phytoalexins, a group of water-soluble phenolic derivatives isomeric with flavonoids that possess antibiotic activity and are produced by plant tissues in response to infection. Also known as: isoflavonoid phytoalexin anabolism, isoflavonoid phytoalexin biosynthesis, isoflavonoid phytoalexin formation, isoflavonoid phytoalexin synthesis Relationships: is a type of isoflavonoid biosynthetic process [GO:0009717]; is_a GO:0052315 Sources: GOC:ai